{
  "term_id": "GO:0004550",
  "gene": "UniProtKB:O75414",
  "term_label": "nucleoside diphosphate kinase activity",
  "gene_name": "Nucleoside diphosphate kinase 6",
  "gene_symbol": "NME6"
}